thyroid-hormone transaminase activity [GO:0033852] (molecular function) Sources: EC:2.6.1.26, RHEA:19133 Definition: Catalysis of the reaction: 2-oxoglutarate + 3,5,3'-triiodo-L-thyronine = 3,5,3'-triiodothyropyruvate + L-glutamate. Also known as: 3,5-dinitrotyrosine aminotransferase activity, 3,5-dinitrotyrosine transaminase activity, L-3,5,3'-triiodothyronine:2-oxoglutarate aminotransferase activity, thyroid hormone aminotransferase activity, thyroid-hormone aminotransferase activity Relationships: is a type of transaminase activity [GO:0008483]